{
  "term_label": "cytoplasm",
  "gene": "UniProtKB:Q96AE4",
  "gene_symbol": "FUBP1",
  "gene_name": "Far upstream element-binding protein 1",
  "term_id": "GO:0005737"
}